{
  "gene_name": "tRNA wybutosine-synthesizing protein 4",
  "term_id": "UNKNOWN:0003",
  "gene": "UniProtKB:O60294",
  "term_label": "Unknown cellular component",
  "gene_symbol": "LCMT2"
}